{
  "gene_symbol": "IL12RB1",
  "term_label": "external side of plasma membrane",
  "term_id": "GO:0009897",
  "gene": "UniProtKB:P42701",
  "gene_name": "Interleukin-12 receptor subunit beta-1"
}